{
  "term_id": "GO:0061630",
  "gene_name": "E3 ubiquitin-protein ligase NRDP1",
  "gene_symbol": "RNF41",
  "term_label": "ubiquitin protein ligase activity",
  "gene": "UniProtKB:Q9H4P4"
}